glycosyl compound catabolic process [GO:1901658] (biological process) Also known as: glycosyl compound breakdown, glycosyl compound catabolism, glycosyl compound degradation Definition: The chemical reactions and pathways resulting in the breakdown of glycosyl compound. Relationships: is a type of GO:1901136 Sources: GOC:TermGenie, GOC:pr Subtypes: GO:0009164, glycoside catabolic process [GO:0016139], GO:0016145